positive regulation of cerebellar neuron development [GO:1905081] (BP) References: PMID:26609159 Sources: GOC:TermGenie, GO_REF:0000058 Definition: Any process that activates or increases the frequency, rate or extent of cerebellar neuron development. Relationships: is_a positive regulation of cell development [GO:0010720]; is a type of GO:0045666; is a type of GO:1905079; positively regulates cerebellar neuron development [GO:0098749] Also known as: up regulation of cerebellar neuron development, up-regulation of cerebellar neuron development, upregulation of cerebellar neuron development, activation of cerebellar neuron development